{
  "gene_name": "Uncharacterized protein C16orf96",
  "term_id": "UNKNOWN:0003",
  "term_label": "Unknown cellular component",
  "gene_symbol": "C16orf96",
  "gene": "UniProtKB:A6NNT2"
}